arugosin biosynthetic process [GO:1900587] (biological process) Also known as: arugosin anabolism, arugosin biosynthesis, arugosin formation, arugosin synthesis Relationships: is a type of secondary metabolite biosynthetic process [GO:0044550] Sources: GOC:TermGenie, GOC:di Definition: The chemical reactions and pathways resulting in the formation of arugosin. Regulation: regulated by regulation of arugosin biosynthetic process [GO:1900626]; negatively regulated by negative regulation of arugosin biosynthetic process [GO:1900627]; RO_0002213 by positive regulation of arugosin biosynthetic process [GO:1900628]